{
  "term_label": "Unknown cellular component",
  "gene_symbol": "ZNF394",
  "gene": "UniProtKB:Q53GI3",
  "term_id": "UNKNOWN:0003",
  "gene_name": "Zinc finger protein 394"
}